'de novo' protein folding [GO:0006458] (biological process) Also known as: nascent chain protein folding Relationships: is a type of protein folding [GO:0006457] Sources: GOC:mb Subtypes: 'de novo' cotranslational protein folding [GO:0051083], 'de novo' post-translational protein folding [GO:0051084] Definition: The process of assisting in the folding of a nascent peptide chain into its correct tertiary structure.